{
  "gene": "UniProtKB:Q5VIR6",
  "gene_symbol": "VPS53",
  "term_label": "retrograde transport, endosome to Golgi",
  "gene_name": "Vacuolar protein sorting-associated protein 53 homolog",
  "term_id": "GO:0042147"
}